{
  "term_label": "fibroblast growth factor receptor binding",
  "gene_name": "Fibroblast growth factor 16",
  "gene_symbol": "FGF16",
  "gene": "UniProtKB:O43320",
  "term_id": "GO:0005104"
}